{
  "gene_symbol": "AK4",
  "term_label": "mitochondrial matrix",
  "term_id": "GO:0005759",
  "gene_name": "Adenylate kinase 4, mitochondrial",
  "gene": "UniProtKB:P27144"
}